{
  "gene": "UniProtKB:O75911",
  "gene_name": "Short-chain dehydrogenase_reductase 3",
  "term_label": "all-trans-retinol dehydrogenase (NAD+) activity",
  "term_id": "GO:0004745",
  "gene_symbol": "DHRS3"
}